{
  "term_label": "exocytic vesicle",
  "gene": "UniProtKB:Q9H2B2",
  "gene_name": "Synaptotagmin-4",
  "term_id": "GO:0070382",
  "gene_symbol": "SYT4"
}